{
  "gene_symbol": "CLDN16",
  "term_id": "GO:0005886",
  "gene_name": "Claudin-16",
  "term_label": "plasma membrane",
  "gene": "UniProtKB:Q9Y5I7"
}